{
  "term_label": "interleukin-11 binding",
  "term_id": "GO:0019970",
  "gene_symbol": "IL11RA",
  "gene_name": "Interleukin-11 receptor subunit alpha",
  "gene": "UniProtKB:Q14626"
}